{
  "gene": "UniProtKB:P53634",
  "gene_symbol": "CTSC",
  "term_label": "extracellular space",
  "term_id": "GO:0005615",
  "gene_name": "Dipeptidyl peptidase 1"
}